negative regulation of neuronal action potential [GO:1904456] (biological process) Definition: Any process that stops, prevents or reduces the frequency, rate or extent of neuronal action potential. Also known as: down regulation of neuronal action potential, down-regulation of neuronal action potential, downregulation of neuronal action potential, inhibition of neuronal action potential, down regulation of generation of action potential, down-regulation of generation of action potential, downregulation of generation of action potential, inhibition of generation of action potential, negative regulation of generation of action potential Relationships: is a type of negative regulation of action potential [GO:0045759]; is a type of negative regulation of transmission of nerve impulse [GO:0051970]; is a type of regulation of neuronal action potential [GO:0098908]; negatively regulates neuronal action potential [GO:0019228] References: PMID:25126967 Sources: GOC:TermGenie, GO_REF:0000058